{
  "term_id": "GO:0036064",
  "gene_symbol": "TTLL4",
  "gene_name": "Tubulin monoglutamylase TTLL4",
  "gene": "UniProtKB:Q14679",
  "term_label": "ciliary basal body"
}